{
  "term_label": "nucleus",
  "gene_name": "RNA exonuclease 1 homolog",
  "gene_symbol": "REXO1",
  "term_id": "GO:0005634",
  "gene": "UniProtKB:Q8N1G1"
}